{
  "gene_symbol": "TGFBRAP1",
  "term_id": "GO:0034058",
  "gene_name": "Transforming growth factor-beta receptor-associated protein 1",
  "gene": "UniProtKB:Q8WUH2",
  "term_label": "endosomal vesicle fusion"
}